{
  "gene_symbol": "SLC6A2",
  "gene_name": "Sodium-dependent noradrenaline transporter",
  "gene": "UniProtKB:P23975",
  "term_id": "GO:0005330",
  "term_label": "dopamine:sodium symporter activity"
}